{
  "term_id": "GO:0043515",
  "gene": "UniProtKB:Q7Z460",
  "gene_symbol": "CLASP1",
  "gene_name": "CLIP-associating protein 1",
  "term_label": "kinetochore binding"
}